Bub1-Bub3 complex localization to kinetochore [GO:1990299] (BP) Definition: A cellular protein complex localization that acts on a Bub1-Bub3 complex; as a result, the complex is transported to, or maintained in, a specific location at the kinetochore. Relationships: is a type of protein-containing complex localization [GO:0031503]; is a type of protein localization to kinetochore [GO:0034501] References: PMID:22521786